{
  "gene_symbol": "A0A0J9YWU9",
  "term_id": "GO:0016064",
  "term_label": "immunoglobulin mediated immune response",
  "gene": "UniProtKB:A0A0J9YWU9",
  "gene_name": "Ig-like domain-containing protein (Fragment)"
}